glycolytic process through fructose-6-phosphate [GO:0061615] (biological process) Also known as: glycolysis through fructose-6-phosphate Subtypes: glycolytic process from fructose through fructose-6-phosphate [GO:0061616], glycolytic process from mannose through fructose-6-phosphate [GO:0061619], GO:0061620, GO:0061706 Definition: The chemical reactions and pathways resulting in the breakdown of a monosaccharide into pyruvate, occurring through a fructose-6-phosphate intermediate, with the concomitant production of ATP and NADH. Relationships: is a type of glycolytic process [GO:0006096]; has part 6-phosphofructokinase activity [GO:0003872]; has part fructose-bisphosphate aldolase activity [GO:0004332]; has part triose-phosphate isomerase activity [GO:0004807] Sources: GOC:dph, ISBN:0201090910, ISBN:0879010479 Regulation: regulated by regulation of glycolytic process through fructose-6-phosphate [GO:1904538]; negatively regulated by negative regulation of glycolytic process through fructose-6-phosphate [GO:1904539]; RO_0002213 by positive regulation of glycolytic process through fructose-6-phosphate [GO:1904540]